{
  "gene": "UniProtKB:Q13489",
  "gene_name": "Baculoviral IAP repeat-containing protein 3",
  "term_id": "GO:0043066",
  "term_label": "negative regulation of apoptotic process",
  "gene_symbol": "BIRC3"
}